positive regulation of cholangiocyte proliferation [GO:1904056] (biological process) Relationships: is a type of positive regulation of epithelial cell proliferation [GO:0050679]; is a type of regulation of cholangiocyte proliferation [GO:1904054]; positively regulates cholangiocyte proliferation [GO:1990705] Also known as: positive regulation of hepatoblast proliferation, up regulation of cholangiocyte proliferation, up regulation of hepatoblast proliferation, up-regulation of cholangiocyte proliferation, up-regulation of hepatoblast proliferation, upregulation of cholangiocyte proliferation, upregulation of hepatoblast proliferation, activation of cholangiocyte proliferation, activation of hepatoblast proliferation Definition: Any process that activates or increases the frequency, rate or extent of cholangiocyte proliferation. References: PMID:24434010 Sources: GOC:TermGenie, GO_REF:0000058